{
  "gene_name": "L-dopachrome tautomerase",
  "term_id": "GO:0048066",
  "term_label": "developmental pigmentation",
  "gene_symbol": "DCT",
  "gene": "UniProtKB:P40126"
}